{
  "gene_symbol": "PLIN2",
  "gene_name": "Perilipin-2",
  "gene": "UniProtKB:Q99541",
  "term_id": "UNKNOWN:0001",
  "term_label": "Unknown molecular function"
}